{
  "gene_symbol": "KIFC2",
  "term_label": "anterograde dendritic transport of neurotransmitter receptor complex",
  "gene": "UniProtKB:Q96AC6",
  "gene_name": "Kinesin-like protein KIFC2",
  "term_id": "GO:0098971"
}